{
  "gene": "UniProtKB:P55854",
  "term_id": "GO:0016925",
  "gene_symbol": "SUMO3",
  "term_label": "protein sumoylation",
  "gene_name": "Small ubiquitin-related modifier 3"
}